{
  "gene": "UniProtKB:Q9H6T3",
  "gene_symbol": "RPAP3",
  "term_id": "UNKNOWN:0001",
  "term_label": "Unknown molecular function",
  "gene_name": "RNA polymerase II-associated protein 3"
}